{
  "term_id": "GO:0090398",
  "gene": "UniProtKB:Q9H1Z8",
  "gene_name": "Augurin",
  "term_label": "cellular senescence",
  "gene_symbol": "ECRG4"
}